{
  "term_label": "Unknown cellular component",
  "gene": "UniProtKB:Q8NDY8",
  "gene_symbol": "TMEM52",
  "term_id": "UNKNOWN:0003",
  "gene_name": "Transmembrane protein 52"
}